phosphinothricin metabolic process [GO:1901764] (biological process) Definition: The chemical reactions and pathways involving phosphinothricin. Subtypes: phosphinothricin catabolic process [GO:1901765], phosphinothricin biosynthetic process [GO:1901766] Also known as: phosphinothricin metabolism Relationships: is a type of GO:0008152 Sources: GOC:TermGenie, GOC:yaf